{
  "term_id": "GO:0006954",
  "gene_name": "Platelet basic protein",
  "gene": "UniProtKB:P02775",
  "gene_symbol": "PPBP",
  "term_label": "inflammatory response"
}